{
  "gene_name": "BOS complex subunit NOMO1",
  "term_id": "UNKNOWN:0001",
  "term_label": "Unknown molecular function",
  "gene": "UniProtKB:Q15155",
  "gene_symbol": "NOMO1"
}